{
  "term_id": "GO:0045948",
  "term_label": "positive regulation of translational initiation",
  "gene_name": "Deleted in azoospermia-like",
  "gene_symbol": "DAZL",
  "gene": "UniProtKB:Q92904"
}